{
  "term_id": "GO:0030970",
  "term_label": "retrograde protein transport, ER to cytosol",
  "gene_name": "Protein OS-9",
  "gene_symbol": "OS9",
  "gene": "UniProtKB:Q13438"
}